{
  "gene_name": "Nesprin-1",
  "term_label": "cytoskeleton-nuclear membrane anchor activity",
  "term_id": "GO:0140444",
  "gene": "UniProtKB:Q8NF91",
  "gene_symbol": "SYNE1"
}